{
  "term_id": "GO:0042373",
  "gene": "UniProtKB:Q8N0U8",
  "term_label": "vitamin K metabolic process",
  "gene_symbol": "VKORC1L1",
  "gene_name": "Vitamin K epoxide reductase complex subunit 1-like protein 1"
}